{
  "term_id": "GO:0004222",
  "gene_name": "A disintegrin and metalloproteinase with thrombospondin motifs 1",
  "term_label": "metalloendopeptidase activity",
  "gene": "UniProtKB:Q9UHI8",
  "gene_symbol": "ADAMTS1"
}